{
  "term_label": "cytoplasm",
  "term_id": "GO:0005737",
  "gene_symbol": "CYP2B6",
  "gene_name": "Cytochrome P450 2B6",
  "gene": "UniProtKB:P20813"
}